{
  "gene": "UniProtKB:P05543",
  "term_id": "GO:0004867",
  "gene_symbol": "SERPINA7",
  "gene_name": "Thyroxine-binding globulin",
  "term_label": "serine-type endopeptidase inhibitor activity"
}